{
  "gene": "UniProtKB:Q9NS68",
  "gene_name": "Tumor necrosis factor receptor superfamily member 19",
  "gene_symbol": "TNFRSF19",
  "term_label": "plasma membrane",
  "term_id": "GO:0005886"
}